{
  "term_label": "RNA polymerase III type 3 promoter sequence-specific DNA binding",
  "term_id": "GO:0001006",
  "gene": "UniProtKB:Q5SXM2",
  "gene_symbol": "SNAPC4",
  "gene_name": "snRNA-activating protein complex subunit 4"
}